{
  "gene": "UniProtKB:Q7Z572",
  "term_id": "UNKNOWN:0002",
  "gene_name": "Spermatogenesis-associated protein 21",
  "gene_symbol": "SPATA21",
  "term_label": "Unknown biological process"
}